negative regulation of amide catabolic process [GO:0034252] (biological process) Definition: Any process that stops, prevents, or reduces the frequency, rate or extent of the chemical reactions and pathways resulting in the breakdown of amides. Subtypes: negative regulation of urea catabolic process [GO:1901713] Relationships: is a type of negative regulation of catabolic process [GO:0009895]; is a type of negative regulation of amide metabolic process [GO:0034249]; is a type of regulation of amide catabolic process [GO:0034251]; negatively regulates amide catabolic process [GO:0043605] Also known as: negative regulation of amide breakdown, negative regulation of amide catabolism, negative regulation of cellular amide catabolic process, negative regulation of amide degradation Sources: GOC:mah